regulation of the velocity of shortening of skeletal muscle modulating contraction [GO:0014729] (biological process) Also known as: regulation of the velocity of shortening of skeletal muscle during contraction Sources: GOC:mtg_muscle Definition: Any process that modulates velocity of shortening of a skeletal muscle contraction. The shortening leads to reduction of the length of muscle fibers and sarcomeres. Relationships: is a type of regulation of skeletal muscle contraction by chemo-mechanical energy conversion [GO:0014862]; is a type of regulation of biological quality [GO:0065008]